{
  "gene_name": "Protein Daple",
  "gene": "UniProtKB:Q9P219",
  "gene_symbol": "CCDC88C",
  "term_id": "GO:0051959",
  "term_label": "dynein light intermediate chain binding"
}